contact chemoreceptor activity [GO:0090684] (MF) Definition: A non-GPCR transmembrane signaling receptor activity that is responsible for contact chemoreception. Sources: GOC:hat, GOC:tb Also known as: contact chemosensation receptor activity Relationships: is a type of taste receptor activity [GO:0008527]